{
  "term_id": "GO:0000978",
  "gene": "UniProtKB:A0A1W2PRP0",
  "gene_name": "Forkhead box protein L3",
  "gene_symbol": "FOXL3",
  "term_label": "RNA polymerase II cis-regulatory region sequence-specific DNA binding"
}